regulation of canonical NF-kappaB signal transduction [GO:0043122] (biological process) Subtypes: positive regulation of canonical NF-kappaB signal transduction [GO:0043123], GO:0043124 References: PMID:12773372 Sources: GOC:jl Also known as: regulation of I-kappaB kinase/NF-kappaB cascade, regulation of I-kappaB kinase/NF-kappaB signaling Relationships: is a type of GO:1902531; regulates canonical NF-kappaB signal transduction [GO:0007249] Definition: Any process that modulates the canonical NF-kappaB signaling cascade.